retrograde dendritic transport of mitochondrion [GO:0098959] (biological process) Sources: GOC:dos Definition: The directed movement of mitochondria along microtubules in dendrites towards the cell body and away from the postsynapse. Relationships: is a type of dendritic transport of mitochondrion [GO:0098939] Also known as: retrograde dendrite transport of mitochondria